vinylacetyl-CoA delta-isomerase activity [GO:0050393] (molecular function) Definition: Catalysis of the reaction: vinylacetyl-CoA = (2E)-butenoyl-CoA. Sources: RHEA:10572 Also known as: delta3-cis-delta2-trans-enoyl-CoA isomerase, vinylacetyl-CoA D-isomerase activity, vinylacetyl coenzyme A delta-isomerase activity, vinylacetyl coenzyme A isomerase activity, vinylacetyl-CoA delta3-delta2-isomerase activity Relationships: is a type of intramolecular oxidoreductase activity, transposing C=C bonds [GO:0016863]